{
  "gene_name": "Serine_threonine-protein kinase Nek8",
  "gene_symbol": "NEK8",
  "term_id": "GO:0005929",
  "gene": "UniProtKB:Q86SG6",
  "term_label": "cilium"
}